azurophil granule membrane [GO:0035577] (cellular component) References: PMID:17152095 Sources: GOC:bf Also known as: primary granule membrane Definition: The lipid bilayer surrounding an azurophil granule, a primary lysosomal granule found in neutrophil granulocytes that contains a wide range of hydrolytic enzymes and is released into the extracellular fluid. Relationships: is_a lysosomal membrane [GO:0005765]; is a type of GO:0030667; is part of azurophil granule [GO:0042582]